{
  "gene_name": "Synaptopodin",
  "term_id": "GO:0001725",
  "gene": "UniProtKB:Q8N3V7",
  "term_label": "stress fiber",
  "gene_symbol": "SYNPO"
}